{
  "gene_name": "Ubiquitin thioesterase otulin",
  "term_id": "GO:0045087",
  "gene": "UniProtKB:Q96BN8",
  "gene_symbol": "OTULIN",
  "term_label": "innate immune response"
}